{
  "gene_name": "Tumor necrosis factor receptor superfamily member 25",
  "gene": "UniProtKB:Q93038",
  "gene_symbol": "TNFRSF25",
  "term_id": "GO:0005886",
  "term_label": "plasma membrane"
}